{
  "gene_name": "Nicotinamide phosphoribosyltransferase",
  "gene": "UniProtKB:P43490",
  "term_label": "nicotinamide phosphoribosyltransferase activity",
  "gene_symbol": "NAMPT",
  "term_id": "GO:0047280"
}